{
  "gene_symbol": "TNFAIP8L2",
  "gene_name": "Tumor necrosis factor alpha-induced protein 8-like protein 2",
  "term_label": "regulation of intracellular signal transduction",
  "term_id": "GO:1902531",
  "gene": "UniProtKB:Q6P589"
}